positive regulation of skeletal muscle acetylcholine-gated channel clustering [GO:1904395] (BP) Definition: Any process that activates or increases the frequency, rate or extent of skeletal muscle acetylcholine-gated channel clustering. Relationships: is a type of positive regulation of receptor clustering [GO:1903911]; is a type of regulation of skeletal muscle acetylcholine-gated channel clustering [GO:1904393]; positively regulates skeletal muscle acetylcholine-gated channel clustering [GO:0071340] References: PMID:7722643 Sources: GOC:TermGenie, GO_REF:0000058 Also known as: positive regulation of skeletal muscle AChR clustering, positive regulation of skeletal muscle nicotinic acetylcholine receptor clustering, up regulation of skeletal muscle AChR clustering, up regulation of skeletal muscle acetylcholine-gated channel clustering, up regulation of skeletal muscle nicotinic acetylcholine receptor clustering, up-regulation of skeletal muscle AChR clustering, up-regulation of skeletal muscle acetylcholine-gated channel clustering, up-regulation of skeletal muscle nicotinic acetylcholine receptor clustering, upregulation of skeletal muscle AChR clustering, upregulation of skeletal muscle acetylcholine-gated channel clustering, upregulation of skeletal muscle nicotinic acetylcholine receptor clustering, activation of skeletal muscle AChR clustering, activation of skeletal muscle acetylcholine-gated channel clustering, activation of skeletal muscle nicotinic acetylcholine receptor clustering